{
  "term_label": "actin cytoskeleton organization",
  "gene_symbol": "SPTBN5",
  "gene_name": "Spectrin beta chain, non-erythrocytic 5",
  "gene": "UniProtKB:Q9NRC6",
  "term_id": "GO:0030036"
}